positive regulation of exocyst assembly [GO:0001930] (biological process) Sources: GOC:hjd Definition: Any process that increases the rate or extent of exocyst assembly. Relationships: is a type of regulation of exocyst assembly [GO:0001928]; is a type of positive regulation of protein-containing complex assembly [GO:0031334]; positively regulates exocyst assembly [GO:0001927] Also known as: up regulation of exocyst assembly, up-regulation of exocyst assembly, upregulation of exocyst assembly, activation of exocyst assembly, stimulation of exocyst assembly